{
  "term_id": "GO:0038111",
  "gene": "UniProtKB:P13232",
  "term_label": "interleukin-7-mediated signaling pathway",
  "gene_name": "Interleukin-7",
  "gene_symbol": "IL7"
}